{
  "gene": "UniProtKB:P62987",
  "term_id": "GO:0031386",
  "gene_symbol": "UBA52",
  "gene_name": "Ubiquitin-ribosomal protein eL40 fusion protein",
  "term_label": "protein tag activity"
}